{
  "gene_name": "Sialidase-4",
  "term_label": "lysosome",
  "gene_symbol": "NEU4",
  "gene": "UniProtKB:Q8WWR8",
  "term_id": "GO:0005764"
}